epithelial cell morphogenesis [GO:0003382] (biological process) Relationships: is a type of cell morphogenesis [GO:0000902]; is part of epithelial cell development [GO:0002064] Sources: GOC:ascb_2009, GOC:dph, GOC:tb Definition: The change in form that occurs when an epithelial cell progresses from its initial formation to its mature state. Subtypes: endothelial cell morphogenesis [GO:0001886], epithelial cell morphogenesis involved in gastrulation [GO:0003381], GO:0060672